mitochondrion-derived vesicle mediated transport [GO:0099075] (biological process) Relationships: is a type of vesicle-mediated transport [GO:0016192] References: PMID:20619655, PMID:37131163 Sources: GOC:PARL-UCL, GOC:bc, GOC:pad Subtypes: GO:0099074, mitochondrion to peroxisome vesicle-mediated transport [GO:0099076] Definition: Vesicle-mediated transport of cargo from the mitochondrion by a mitochondrion-derived vesicle.